{
  "gene_name": "Transmembrane protein 31",
  "term_label": "Unknown biological process",
  "gene_symbol": "TMEM31",
  "term_id": "UNKNOWN:0002",
  "gene": "UniProtKB:Q5JXX7"
}